{
  "gene": "UniProtKB:P50993",
  "gene_symbol": "ATP1A2",
  "term_id": "GO:1902600",
  "gene_name": "Sodium_potassium-transporting ATPase subunit alpha-2",
  "term_label": "proton transmembrane transport"
}